{
  "gene_name": "Dexamethasone-induced protein",
  "gene": "UniProtKB:O95424",
  "term_id": "UNKNOWN:0001",
  "gene_symbol": "DEXI",
  "term_label": "Unknown molecular function"
}